response to mitotic G2 DNA damage checkpoint signaling [GO:0072435] (BP) Definition: A process that occurs in response to signals generated as a result of mitotic G2/M transition DNA damage checkpoint signaling. Also known as: mitotic G2/M transition DNA damage checkpoint effector process, response to mitotic G2/M transition DNA damage checkpoint signaling, response to signal involved in mitotic G2/M transition DNA damage checkpoint, mitotic G2/M transition decatenation checkpoint effector process, response to mitotic G2/M transition decatenation checkpoint signaling, response to signal involved in mitotic G2/M transition decatenation checkpoint Relationships: is a type of GO:0072414; is a type of response to G2 DNA damage checkpoint signaling [GO:0072426] Sources: GOC:mtg_cell_cycle